{
  "term_id": "UNKNOWN:0001",
  "term_label": "Unknown molecular function",
  "gene_name": "Active breakpoint cluster region-related protein",
  "gene": "UniProtKB:Q12979",
  "gene_symbol": "ABR"
}